mucosal lymphocyte homeostasis [GO:0002261] (biological process) References: PMID:15609020 Sources: GOC:add Relationships: is a type of lymphocyte homeostasis [GO:0002260] Definition: The process of regulating the proliferation and elimination of lymphocytes such that the total number of lymphocytes within the mucosal tissue of an organism is stable over time in the absence of an outside stimulus.